{
  "gene": "UniProtKB:Q8NC06",
  "gene_name": "Acyl-CoA-binding domain-containing protein 4",
  "gene_symbol": "ACBD4",
  "term_label": "cytoplasm",
  "term_id": "GO:0005737"
}